regulation of translation at postsynapse, modulating synaptic transmission [GO:0099578] (biological process) Definition: Any process that modulates synaptic transmission by regulating translation occurring at the postsynapse. Relationships: is a type of postsynaptic modulation of chemical synaptic transmission [GO:0099170]; is a type of regulation of translation at synapse, modulating synaptic transmission [GO:0099547]; is a type of regulation of translation at postsynapse [GO:0140245] Note: Note that this term was created for the SynGO project, and will be obsoleted when the SynGO annotations are made in Noctua. Sources: GOC:dos